ABC-type choline transporter activity [GO:0033266] (molecular function) Relationships: is a type of choline transmembrane transporter activity [GO:0015220]; is a type of ABC-type transporter activity [GO:0140359] Also known as: ABC-type choline transmembrane transporter activity, ATP-dependent choline transmembrane transporter activity, ATPase-coupled choline transmembrane transporter activity, choline-transporting ATPase activity Sources: GOC:mlg Definition: Catalysis of the reaction: ATP + H2O = ADP + phosphate, to directly drive the transport of choline across a membrane.